{
  "gene": "UniProtKB:Q8N2U9",
  "gene_name": "Solute carrier family 66 member 2",
  "gene_symbol": "SLC66A2",
  "term_label": "Unknown molecular function",
  "term_id": "UNKNOWN:0001"
}